{
  "term_id": "GO:0005737",
  "gene_symbol": "MYH1",
  "gene": "UniProtKB:P12882",
  "gene_name": "Myosin-1",
  "term_label": "cytoplasm"
}